{
  "gene_name": "Protein FAM110C",
  "term_label": "positive regulation of cell migration",
  "gene": "UniProtKB:Q1W6H9",
  "term_id": "GO:0030335",
  "gene_symbol": "FAM110C"
}